{
  "term_label": "external side of plasma membrane",
  "gene": "UniProtKB:Q13291",
  "gene_symbol": "SLAMF1",
  "term_id": "GO:0009897",
  "gene_name": "Signaling lymphocytic activation molecule"
}